{
  "gene_symbol": "NNMT",
  "gene": "UniProtKB:P40261",
  "term_label": "nicotinamide N-methyltransferase activity",
  "gene_name": "Nicotinamide N-methyltransferase",
  "term_id": "GO:0008112"
}